{
  "gene_name": "Scavenger receptor class A member 5",
  "term_id": "GO:0005044",
  "term_label": "scavenger receptor activity",
  "gene": "UniProtKB:Q6ZMJ2",
  "gene_symbol": "SCARA5"
}